{
  "gene_name": "Ras-related protein Rap-2c",
  "gene": "UniProtKB:Q9Y3L5",
  "term_label": "negative regulation of cell migration",
  "gene_symbol": "RAP2C",
  "term_id": "GO:0030336"
}